{
  "gene": "UniProtKB:O95633",
  "gene_name": "Follistatin-related protein 3",
  "gene_symbol": "FSTL3",
  "term_id": "GO:0005576",
  "term_label": "extracellular region"
}